negative regulation of response to furfural [GO:1901443] (biological process) Also known as: down regulation of response to furfural, down-regulation of response to furfural, downregulation of response to furfural, inhibition of response to furfural Relationships: is a type of negative regulation of response to stimulus [GO:0048585]; is a type of regulation of response to furfural [GO:1901442]; negatively regulates GO:1901426 Sources: GOC:TermGenie, GOC:mengo_curators Definition: Any process that stops, prevents or reduces the frequency, rate or extent of response to furfural.